fatty acid transmembrane transporter activity [GO:0015245] (molecular function) Sources: ISBN:0198506732 Subtypes: GO:0005324, short-chain fatty acid transmembrane transporter activity [GO:0015636], beta-hydroxybutyrate transmembrane transporter activity [GO:0097253] Also known as: fatty-acyl group transporter activity, fatty acyl transporter activity, peroxisomal fatty acyl transporter, fatty acid transporter activity Relationships: is a type of GO:0008028; is_a lipid transmembrane transporter activity [GO:0170055]; is part of GO:0015908 Definition: Enables the transfer of fatty acids from one side of a membrane to the other. Fatty acids are aliphatic monocarboxylic acids liberated from naturally occurring fats and oils by hydrolysis.